sensory perception of smell [GO:0007608] (biological process) Definition: The series of events required for an organism to receive an olfactory stimulus, convert it to a molecular signal, and recognize and characterize the signal. Olfaction involves the detection of chemical composition of an organism's ambient medium by chemoreceptors. This is a neurological process. Relationships: is_a GO:0007606 Sources: GOC:ai Also known as: olfaction, scent perception, sense of smell, smell perception